{
  "term_id": "UNKNOWN:0003",
  "gene_symbol": "TTC39A",
  "gene_name": "Tetratricopeptide repeat protein 39A",
  "term_label": "Unknown cellular component",
  "gene": "UniProtKB:Q5SRH9"
}